{
  "gene_name": "Large ribosomal subunit protein bL33m",
  "term_label": "mitochondrion",
  "gene_symbol": "MRPL33",
  "gene": "UniProtKB:O75394",
  "term_id": "GO:0005739"
}